{
  "gene_name": "Putative upstream-binding factor 1-like protein 6",
  "gene_symbol": "UBTFL6",
  "term_label": "RNA polymerase I general transcription initiation factor activity",
  "term_id": "GO:0001181",
  "gene": "UniProtKB:P0CB48"
}